{
  "gene_symbol": "TMEM178A",
  "gene": "UniProtKB:Q8NBL3",
  "term_id": "GO:0051480",
  "gene_name": "Transmembrane protein 178A",
  "term_label": "regulation of cytosolic calcium ion concentration"
}